nucleotide-excision repair factor 1 complex [GO:0000110] (cellular component) Also known as: NEF1 complex, XPA-ERCC1-ERCC4 complex Note: Note that process and function information are included in the term and definition for the purpose of describing and distinguishing the complex. Definition: One of several protein complexes involved in nucleotide-excision repair; possesses DNA damage recognition and endodeoxynuclease activities. In S. cerevisiae, it is composed of Rad1p, Rad10p, and Rad14p; in human the subunits are ERCC4/XPF, ERCC1 and XPA, respectively. References: PMID:10915862 Relationships: is a type of nucleotide-excision repair complex [GO:0000109]